positive regulation of toll-like receptor 15 signaling pathway [GO:2000442] (BP) Definition: Any process that activates or increases the frequency, rate or extent of toll-like receptor 15 signaling pathway. Sources: GOC:obol Relationships: is a type of GO:0062208; is a type of regulation of toll-like receptor 15 signaling pathway [GO:2000440]; positively regulates toll-like receptor 15 signaling pathway [GO:0035681] Also known as: positive regulation of TLR15 signaling pathway, positive regulation of toll-like receptor 15 signalling pathway